{
  "gene_symbol": "PPIL4",
  "gene": "UniProtKB:Q8WUA2",
  "gene_name": "Peptidyl-prolyl cis-trans isomerase-like 4",
  "term_label": "Unknown biological process",
  "term_id": "UNKNOWN:0002"
}